{
  "gene_symbol": "OR8B2",
  "term_id": "UNKNOWN:0003",
  "gene": "UniProtKB:Q96RD0",
  "gene_name": "Olfactory receptor 8B2",
  "term_label": "Unknown cellular component"
}